{
  "gene_name": "POM121-like protein 2",
  "gene_symbol": "POM121L2",
  "gene": "UniProtKB:Q96KW2",
  "term_label": "protein import into nucleus",
  "term_id": "GO:0006606"
}